{
  "gene": "UniProtKB:Q8NCW0",
  "gene_symbol": "KREMEN2",
  "gene_name": "Kremen protein 2",
  "term_label": "signal transduction",
  "term_id": "GO:0007165"
}